{
  "term_id": "UNKNOWN:0003",
  "gene_symbol": "CCDC194",
  "gene_name": "Coiled-coil domain-containing protein 194",
  "gene": "UniProtKB:A0A1B0GVG4",
  "term_label": "Unknown cellular component"
}